response to tropane [GO:0014073] (biological process) Sources: GOC:ef Definition: Any process that results in a change in state or activity of a cell or an organism (in terms of movement, secretion, enzyme production, gene expression, etc.) as a result of a tropane stimulus. Tropane is a nitrogenous bicyclic organic compound mainly known for a group of alkaloids derived from it (called tropane alkaloids), which include, among others, atropine and cocaine. Subtypes: GO:0071416 Relationships: is a type of GO:0043279